regulation of glucocorticoid secretion [GO:2000849] (biological process) Definition: Any process that modulates the frequency, rate or extent of glucocorticoid secretion. Sources: GOC:sl Relationships: is a type of regulation of corticosteroid hormone secretion [GO:2000846]; regulates glucocorticoid secretion [GO:0035933] Subtypes: regulation of cortisol secretion [GO:0051462], GO:2000850, positive regulation of glucocorticoid secretion [GO:2000851], regulation of corticosterone secretion [GO:2000852]